{
  "term_id": "GO:0000122",
  "gene": "UniProtKB:Q9HCK0",
  "gene_name": "Zinc finger and BTB domain-containing protein 26",
  "gene_symbol": "ZBTB26",
  "term_label": "negative regulation of transcription by RNA polymerase II"
}